{
  "term_label": "response to lipopolysaccharide",
  "gene_symbol": "NOS3",
  "term_id": "GO:0032496",
  "gene_name": "Nitric oxide synthase 3",
  "gene": "UniProtKB:P29474"
}